energy derivation by oxidation of organic compounds [GO:0015980] (biological process) Also known as: chemoorganotrophy Sources: GOC:mah Relationships: is a type of generation of precursor metabolites and energy [GO:0006091] Subtypes: energy reserve metabolic process [GO:0006112], fermentation [GO:0006113], cellular respiration [GO:0045333] Definition: The chemical reactions and pathways by which a cell derives energy from organic compounds; results in the oxidation of the compounds from which energy is released.